non-canonical NF-kappaB signal transduction [GO:0038061] (biological process) References: PMID:11239468, PMID:15140882, PMID:34659217 Sources: GOC:bf, GOC:mg2, GOC:signaling, GOC:vs Relationships: is a type of intracellular signaling cassette [GO:0141124] Regulation: regulated by regulation of non-canonical NF-kappaB signal transduction [GO:1901222]; RO_0002212 by GO:1901223; positively regulated by positive regulation of non-canonical NF-kappaB signal transduction [GO:1901224] Also known as: NF-kappaB cascade, NIK-IKK kinase cascade, NIK-IKK signaling pathway, NIK-IKK-alpha cascade, NIK/NF-kappaB cascade, NIK/NF-kappaB signal transduction, NIK/NF-kappaB signaling, non-canonical NF-KB signaling, noncanonical NF-kappaB signaling, noncanonical nuclear factor kappaB (NF-kappaB) pathway, p52-dependent NF-kappaB signaling Definition: An intracellular signaling cassette characterized by the NIK-dependent processing and activation of NF-kappaB. Begins with activation of the NF-kappaB-inducing kinase (NIK), which in turn phosphorylates and activates IkappaB kinase alpha (IKKalpha). IKKalpha phosphorylates the NF-kappa B2 protein (p100) leading to p100 processing and release of an active NF-kappaB (p52). The non-canonical NF-kappaB signaling pathway is generally activated by ligands of the TNF receptor superfamily, including lymphotoxin beta (LTB), CD40, OX40, RANK, TWEAK and B cell-activating factor (BAFF).